{
  "term_label": "Unknown biological process",
  "term_id": "UNKNOWN:0002",
  "gene": "UniProtKB:Q6ZTC4",
  "gene_name": "Putative uncharacterized protein FLJ44790",
  "gene_symbol": "Q6ZTC4"
}